{
  "term_id": "UNKNOWN:0002",
  "term_label": "Unknown biological process",
  "gene_symbol": "ZMYM4",
  "gene_name": "Zinc finger MYM-type protein 4",
  "gene": "UniProtKB:Q5VZL5"
}